{
  "gene": "UniProtKB:Q8IV36",
  "term_label": "Unknown molecular function",
  "gene_name": "Protein HID1",
  "term_id": "UNKNOWN:0001",
  "gene_symbol": "HID1"
}